anoikis [GO:0043276] (biological process) References: PMID:37667281 Sources: GOC:jl Definition: Apoptosis triggered by inadequate or inappropriate adherence to substrate e.g. after disruption of the interactions between normal epithelial cells and the extracellular matrix. Also known as: detachment induced cell death, suspension induced apoptosis Relationships: is a type of apoptotic process [GO:0006915] Regulation: regulated by regulation of anoikis [GO:2000209]; positively regulated by positive regulation of anoikis [GO:2000210]; RO_0002212 by negative regulation of anoikis [GO:2000811]